{
  "term_label": "cell surface",
  "gene": "UniProtKB:Q86YC3",
  "gene_name": "Transforming growth factor beta activator LRRC33",
  "gene_symbol": "NRROS",
  "term_id": "GO:0009986"
}